pharyngeal arch artery morphogenesis [GO:0061626] (biological process) Definition: The process in which the anatomical structures of a pharyngeal arch artery is generated and organized. The pharyngeal arch arteries are a series of six paired embryological vascular structures, the development of which give rise to several major arteries, such as the stapedial artery, the middle meningeal artery, the internal carotid artery and the pulmonary artery. Also known as: aortic arch artery morphogenesis References: PMID:20122914 Sources: GOC:BHF, GOC:dph Relationships: is a type of artery morphogenesis [GO:0048844]; BFO_0000050 GO:0060037